{
  "gene_name": "Nucleoplasmin-2",
  "term_id": "GO:0003723",
  "gene_symbol": "NPM2",
  "term_label": "RNA binding",
  "gene": "UniProtKB:Q86SE8"
}